{
  "term_id": "UNKNOWN:0003",
  "gene_symbol": "GIPC1",
  "term_label": "Unknown cellular component",
  "gene_name": "PDZ domain-containing protein GIPC1",
  "gene": "UniProtKB:O14908"
}